{
  "term_id": "GO:0001708",
  "gene_symbol": "APC2",
  "gene": "UniProtKB:O95996",
  "gene_name": "Adenomatous polyposis coli protein 2",
  "term_label": "cell fate specification"
}